{
  "gene_symbol": "CCR5",
  "gene": "UniProtKB:P51681",
  "term_id": "GO:0071791",
  "term_label": "chemokine (C-C motif) ligand 5 binding",
  "gene_name": "C-C chemokine receptor type 5"
}